{
  "term_id": "GO:0009897",
  "gene": "UniProtKB:Q6UXB4",
  "gene_symbol": "CLEC4G",
  "term_label": "external side of plasma membrane",
  "gene_name": "C-type lectin domain family 4 member G"
}